{
  "term_id": "GO:0030198",
  "gene": "UniProtKB:Q9ULZ9",
  "gene_symbol": "MMP17",
  "term_label": "extracellular matrix organization",
  "gene_name": "Matrix metalloproteinase-17"
}